{
  "gene_name": "Angiopoietin-1 receptor",
  "term_id": "GO:0043410",
  "gene_symbol": "TEK",
  "gene": "UniProtKB:Q02763",
  "term_label": "positive regulation of MAPK cascade"
}